{
  "term_label": "Unknown molecular function",
  "gene_symbol": "SCYGR5",
  "gene_name": "Small cysteine and glycine repeat-containing protein 5",
  "gene": "UniProtKB:A0A286YF46",
  "term_id": "UNKNOWN:0001"
}